{
  "term_label": "guanyl-nucleotide exchange factor activity",
  "gene_symbol": "KALRN",
  "term_id": "GO:0005085",
  "gene": "UniProtKB:O60229",
  "gene_name": "Kalirin"
}